bidirectional double-stranded viral DNA replication [GO:0039686] (biological process) Relationships: is a type of viral DNA genome replication [GO:0039693] Definition: A viral DNA replication process where replication occurs in both directions from the starting point. This creates two replication forks, moving in opposite directions. Also known as: viral bidirectional dsDNA replication Sources: GOC:bf, GOC:jl, VZ:1939